{
  "term_label": "Unknown biological process",
  "term_id": "UNKNOWN:0002",
  "gene_name": "Small G protein signaling modulator 1",
  "gene": "UniProtKB:Q2NKQ1",
  "gene_symbol": "SGSM1"
}